{
  "term_label": "melanosome membrane",
  "gene": "UniProtKB:Q9UMX9",
  "gene_name": "Membrane-associated transporter protein",
  "term_id": "GO:0033162",
  "gene_symbol": "SLC45A2"
}